{
  "term_label": "cytokine-mediated signaling pathway",
  "term_id": "GO:0019221",
  "gene_name": "Interleukin-31 receptor subunit alpha",
  "gene": "UniProtKB:Q8NI17",
  "gene_symbol": "IL31RA"
}